{
  "term_label": "adenylate cyclase-modulating G protein-coupled receptor signaling pathway",
  "gene": "UniProtKB:O95838",
  "gene_symbol": "GLP2R",
  "term_id": "GO:0007188",
  "gene_name": "Glucagon-like peptide 2 receptor"
}